{
  "gene_name": "Endothelin-1",
  "term_label": "endothelin B receptor binding",
  "gene": "UniProtKB:P05305",
  "term_id": "GO:0031708",
  "gene_symbol": "EDN1"
}